{
  "term_label": "extracellular region",
  "term_id": "GO:0005576",
  "gene": "UniProtKB:Q6WRI0",
  "gene_symbol": "IGSF10",
  "gene_name": "Immunoglobulin superfamily member 10"
}